{
  "term_id": "UNKNOWN:0002",
  "gene": "UniProtKB:Q02747",
  "gene_symbol": "GUCA2A",
  "term_label": "Unknown biological process",
  "gene_name": "Guanylin"
}